{
  "gene_symbol": "E2F7",
  "gene": "UniProtKB:Q96AV8",
  "term_id": "GO:0006357",
  "gene_name": "Transcription factor E2F7",
  "term_label": "regulation of transcription by RNA polymerase II"
}